{
  "term_id": "GO:0017069",
  "gene_name": "Target of EGR1 protein 1",
  "gene": "UniProtKB:Q96GM8",
  "gene_symbol": "TOE1",
  "term_label": "snRNA binding"
}